{
  "gene_name": "POTE ankyrin domain family member I",
  "term_label": "structural constituent of postsynaptic actin cytoskeleton",
  "gene_symbol": "POTEI",
  "gene": "UniProtKB:P0CG38",
  "term_id": "GO:0098973"
}